negative regulation of activated CD4-positive, alpha-beta T cell apoptotic process [GO:1905400] (biological process) Relationships: is a type of negative regulation of T cell apoptotic process [GO:0070233]; is a type of regulation of activated CD4-positive, alpha-beta T cell apoptotic process [GO:1905399]; negatively regulates activated CD4-positive, alpha-beta T cell apoptotic process [GO:1905398] Definition: Any process that stops, prevents or reduces the frequency, rate or extent of activated CD4-positive, alpha-beta T cell apoptotic process. References: PMID:24187568 Sources: GOC:TermGenie, GO_REF:0000058 Also known as: down regulation of activated CD4-positive, alpha-beta T cell apoptotic process, down regulation of activated CD4-positive, alpha-beta T lymphocyte apoptotic process, down regulation of activated CD4-positive, alpha-beta T-cell apoptotic process, down regulation of activated CD4-positive, alpha-beta T-lymphocyte apoptotic process, down-regulation of activated CD4-positive, alpha-beta T cell apoptotic process, down-regulation of activated CD4-positive, alpha-beta T lymphocyte apoptotic process, down-regulation of activated CD4-positive, alpha-beta T-cell apoptotic process, down-regulation of activated CD4-positive, alpha-beta T-lymphocyte apoptotic process, downregulation of activated CD4-positive, alpha-beta T cell apoptotic process, downregulation of activated CD4-positive, alpha-beta T lymphocyte apoptotic process, downregulation of activated CD4-positive, alpha-beta T-cell apoptotic process, downregulation of activated CD4-positive, alpha-beta T-lymphocyte apoptotic process, negative regulation of activated CD4-positive, alpha-beta T lymphocyte apoptotic process, negative regulation of activated CD4-positive, alpha-beta T-cell apoptotic process, negative regulation of activated CD4-positive, alpha-beta T-lymphocyte apoptotic process, down regulation of activated CD4-positive, alpha-beta T cell apoptosis, down regulation of activated CD4-positive, alpha-beta T lymphocyte apoptosis, down regulation of activated CD4-positive, alpha-beta T-cell apoptosis, down regulation of activated CD4-positive, alpha-beta T-lymphocyte apoptosis, down-regulation of activated CD4-positive, alpha-beta T cell apoptosis, down-regulation of activated CD4-positive, alpha-beta T lymphocyte apoptosis, down-regulation of activated CD4-positive, alpha-beta T-cell apoptosis, down-regulation of activated CD4-positive, alpha-beta T-lymphocyte apoptosis, downregulation of activated CD4-positive, alpha-beta T cell apoptosis, downregulation of activated CD4-positive, alpha-beta T lymphocyte apoptosis, downregulation of activated CD4-positive, alpha-beta T-cell apoptosis, downregulation of activated CD4-positive, alpha-beta T-lymphocyte apoptosis, inhibition of activated CD4-positive, alpha-beta T cell apoptosis, inhibition of activated CD4-positive, alpha-beta T cell apoptotic process, inhibition of activated CD4-positive, alpha-beta T lymphocyte apoptosis, inhibition of activated CD4-positive, alpha-beta T lymphocyte apoptotic process, inhibition of activated CD4-positive, alpha-beta T-cell apoptosis, inhibition of activated CD4-positive, alpha-beta T-cell apoptotic process, inhibition of activated CD4-positive, alpha-beta T-lymphocyte apoptosis, inhibition of activated CD4-positive, alpha-beta T-lymphocyte apoptotic process, negative regulation of activated CD4-positive, alpha-beta T cell apoptosis, negative regulation of activated CD4-positive, alpha-beta T lymphocyte apoptosis, negative regulation of activated CD4-positive, alpha-beta T-cell apoptosis, negative regulation of activated CD4-positive, alpha-beta T-lymphocyte apoptosis